{
  "gene": "UniProtKB:Q9P275",
  "gene_symbol": "USP36",
  "term_label": "nucleus",
  "term_id": "GO:0005634",
  "gene_name": "Ubiquitin carboxyl-terminal hydrolase 36"
}